copper ion import [GO:0015677] (biological process) Definition: The directed movement of copper ions into a cell or organelle. Sources: GOC:ai Also known as: copper ion uptake Relationships: is_a GO:0006825